sperm competition [GO:0046692] (BP) Subtypes: GO:0007321, sperm storage [GO:0046693], sperm incapacitation [GO:0046694] References: PMID:10885514 Relationships: is a type of GO:0044703; is a type of multi-multicellular organism process [GO:0044706]; is a type of GO:0048609; is part of insemination [GO:0007320] Definition: Any process that contributes to the success of sperm fertilization in multiply-mated females.